{
  "gene_symbol": "RIMBP3",
  "gene": "UniProtKB:Q9UFD9",
  "term_id": "GO:0009566",
  "gene_name": "RIMS-binding protein 3A",
  "term_label": "fertilization"
}